{
  "gene_name": "Inward rectifier potassium channel 13",
  "term_label": "Unknown molecular function",
  "term_id": "UNKNOWN:0001",
  "gene_symbol": "KCNJ13",
  "gene": "UniProtKB:O60928"
}